{
  "term_id": "GO:0019901",
  "gene": "UniProtKB:Q96EL1",
  "gene_symbol": "INKA1",
  "gene_name": "PAK4-inhibitor INKA1",
  "term_label": "protein kinase binding"
}